exo-oligoalginate lyase activity [GO:0052764] (molecular function) Relationships: is a type of carbon-oxygen lyase activity, acting on polysaccharides [GO:0016837] References: PMID:20925655 Sources: GOC:mengo_curators Definition: Catalysis of the cleavage of glycosidic bonds through a beta-elimination reaction on alginate, a linear polysaccharide consisting of guluronate (G) and mannuronate (M) as the monomer constituents. An oligoalginate is a linear polymer of two, three or four units of (1->4)-alpha-L-guluronic acid and beta-D-mannuronic acid, releasing monosaccharides with 4-deoxy-alpha-L-erythro-hex-4-enopyranuronosyl groups at their ends.